{
  "term_label": "cytoskeleton",
  "gene_symbol": "RHOBTB1",
  "gene_name": "Rho-related BTB domain-containing protein 1",
  "term_id": "GO:0005856",
  "gene": "UniProtKB:O94844"
}